{
  "term_id": "GO:0007204",
  "gene": "UniProtKB:Q86UU9",
  "gene_name": "Tachykinin-4",
  "gene_symbol": "TAC4",
  "term_label": "positive regulation of cytosolic calcium ion concentration"
}